regulation of inflammatory response to wounding [GO:0106014] (BP) Definition: Any process that modulates the frequency, rate or extent of the inflammatory response to wounding. Relationships: is_a regulation of inflammatory response [GO:0050727]; is a type of GO:1903034; regulates GO:0090594 References: PMID:26022821 Sources: GOC:BHF, GOC:BHF_miRNA, GOC:rph Subtypes: negative regulation of inflammatory response to wounding [GO:0106015], GO:0106016